DNA endonuclease activity [GO:0004520] (molecular function) Regulation: regulated by GO:0032071; positively regulated by GO:0032079; positively regulated by GO:0140656 Relationships: is a type of endonuclease activity [GO:0004519]; is a type of GO:0004536 Also known as: endodeoxyribonuclease activity, DNA nicking activity, endonuclease G activity Sources: GOC:mah, ISBN:0198547684 Subtypes: single-stranded DNA endodeoxyribonuclease activity [GO:0000014], GO:0003906, GO:0009381, restriction endodeoxyribonuclease activity [GO:0015666], GO:0016888, DNA endonuclease activity, producing 3'-phosphomonoesters [GO:0016889], GO:0033892, T/G mismatch-specific endonuclease activity [GO:0043765], GO:0044824, GO:0048256, double-stranded DNA endonuclease activity [GO:1990238] Definition: Catalysis of the cleavage of ester linkages within deoxyribonucleic acid by creating internal breaks.